{
  "term_id": "GO:0051156",
  "term_label": "glucose 6-phosphate metabolic process",
  "gene_symbol": "GPI",
  "gene_name": "Glucose-6-phosphate isomerase",
  "gene": "UniProtKB:P06744"
}